{
  "gene_name": "DBIRD complex subunit ZNF326",
  "gene": "UniProtKB:Q5BKZ1",
  "term_label": "Unknown molecular function",
  "gene_symbol": "ZNF326",
  "term_id": "UNKNOWN:0001"
}